{
  "term_label": "Unknown molecular function",
  "gene_name": "Centromere protein V-like protein 2",
  "term_id": "UNKNOWN:0001",
  "gene": "UniProtKB:P0DPI3",
  "gene_symbol": "CENPVL2"
}